sterol transfer activity [GO:0120015] (molecular function) Also known as: sterol carrier activity, intermembrane sterol transfer activity References: PMID:20823909, PMID:24220498, PMID:25797198 Sources: GOC:krc Definition: Removes a sterol from a membrane or a monolayer lipid particle, transports it through the aqueous phase while protected in a hydrophobic pocket, and brings it to an acceptor membrane or lipid particle. Subtypes: cholesterol transfer activity [GO:0120020], GO:0120021 Relationships: is a type of GO:0120013; is part of sterol transport [GO:0015918]; has part sterol binding [GO:0032934]